{
  "gene": "UniProtKB:Q9BYC2",
  "term_label": "mitochondrion",
  "gene_name": "Succinyl-CoA:3-ketoacid coenzyme A transferase 2, mitochondrial",
  "term_id": "GO:0005739",
  "gene_symbol": "OXCT2"
}